{
  "term_id": "GO:0003723",
  "gene_name": "Regulator of nonsense transcripts 1",
  "gene": "UniProtKB:Q92900",
  "term_label": "RNA binding",
  "gene_symbol": "UPF1"
}